{
  "term_label": "kidney morphogenesis",
  "gene_symbol": "NPHP3",
  "term_id": "GO:0060993",
  "gene": "UniProtKB:Q7Z494",
  "gene_name": "Nephrocystin-3"
}